steroid biosynthetic process [GO:0006694] (biological process) Subtypes: sterol biosynthetic process [GO:0016126], phytosteroid biosynthetic process [GO:0016129], vitamin D biosynthetic process [GO:0042368], ecdysteroid biosynthetic process [GO:0045456], testosterone biosynthetic process [GO:0061370], brexanolone biosynthetic process [GO:0062174], steroid hormone biosynthetic process [GO:0120178], andrastin A biosynthetic process [GO:0140876], (17Z)-protosta-17(20),24-dien-3beta-ol biosynthetic process [GO:1900581], helvolic acid biosynthetic process [GO:1900812], androst-4-ene-3,17-dione biosynthetic process [GO:1903449], ergosteryl 3-beta-D-glucoside biosynthetic process [GO:1904463] Regulation: positively regulated by positive regulation of steroid biosynthetic process [GO:0010893]; RO_0002212 by GO:0010894; regulated by GO:0050810 Relationships: is a type of steroid metabolic process [GO:0008202]; is a type of GO:0008610 Sources: GOC:go_curators Also known as: steroid anabolism, steroid biosynthesis, steroid formation, steroid synthesis, steroidogenesis Definition: The chemical reactions and pathways resulting in the formation of steroids, compounds with a 1,2,cyclopentanoperhydrophenanthrene nucleus; includes de novo formation and steroid interconversion by modification.